{
  "gene_symbol": "RAB32",
  "term_label": "melanosome",
  "gene": "UniProtKB:Q13637",
  "gene_name": "Ras-related protein Rab-32",
  "term_id": "GO:0042470"
}